{
  "term_label": "Unknown molecular function",
  "gene_symbol": "FNDC10",
  "term_id": "UNKNOWN:0001",
  "gene": "UniProtKB:F2Z333",
  "gene_name": "Fibronectin type III domain-containing protein 10"
}